nutrient reservoir activity [GO:0045735] (molecular function) Definition: Functions in the storage of nutritious substrates. Relationships: is a type of molecular_function [GO:0003674] Sources: GOC:ai Note: Note that this term can be used in place of the obsolete terms 'storage protein ; GO:0005187' and 'storage protein of fat body (sensu Insecta) ; GO:0008041'. Also known as: storage protein, storage protein of fat body, yolk protein